{
  "term_label": "transmembrane transporter binding",
  "gene_name": "Voltage-dependent calcium channel beta subunit-associated regulatory protein",
  "term_id": "GO:0044325",
  "gene_symbol": "CBARP",
  "gene": "UniProtKB:Q8N350"
}